cochlear hair cell ribbon synapse [GO:0098683] (cellular component) Definition: A ribbon synpase of an auditory hair cell of the cochlear. These ribbon synapses contain spherical synaptic ribbons and lack and arciform density. References: PMID:15626493 Relationships: is a type of GO:0097470